{
  "gene_name": "Serine_threonine-protein kinase PAK 1",
  "term_label": "regulation of actin cytoskeleton organization",
  "gene_symbol": "PAK1",
  "term_id": "GO:0032956",
  "gene": "UniProtKB:Q13153"
}